{
  "gene_name": "Homeodomain-interacting protein kinase 3",
  "term_id": "GO:0004674",
  "gene": "UniProtKB:Q9H422",
  "gene_symbol": "HIPK3",
  "term_label": "protein serine/threonine kinase activity"
}